{
  "gene_name": "Proteasome subunit alpha-type 8",
  "term_id": "UNKNOWN:0001",
  "term_label": "Unknown molecular function",
  "gene": "UniProtKB:Q8TAA3",
  "gene_symbol": "PSMA8"
}